very-low-density lipoprotein particle clearance [GO:0034447] (biological process) Definition: The process in which a very-low-density lipoprotein particle is removed from the blood via receptor-mediated endocytosis and its constituent parts degraded. Relationships: is a type of GO:0034381 Sources: GOC:BHF, GOC:rl Also known as: VLDL clearance Regulation: regulated by regulation of very-low-density lipoprotein particle clearance [GO:0010915]; negatively regulated by negative regulation of very-low-density lipoprotein particle clearance [GO:0010916]; positively regulated by GO:0110119